alpha-beta T cell lineage commitment [GO:0002363] (biological process) Relationships: is a type of T cell lineage commitment [GO:0002360]; is part of GO:0046632 Sources: GOC:add, ISBN:0781735149 Subtypes: GO:0002364, CD4-positive, alpha-beta T cell lineage commitment [GO:0043373], CD8-positive, alpha-beta T cell lineage commitment [GO:0043375] Definition: The process in which a pro-T cell becomes committed to becoming an alpha-beta T cell. Also known as: alpha-beta T lymphocyte lineage commitment, alpha-beta T-cell lineage commitment, alpha-beta T-lymphocyte lineage commitment